{
  "gene_symbol": "ZBTB48",
  "term_id": "GO:0006357",
  "gene": "UniProtKB:P10074",
  "term_label": "regulation of transcription by RNA polymerase II",
  "gene_name": "Telomere zinc finger-associated protein"
}